{
  "gene_name": "Kallikrein-4",
  "term_label": "secretory granule",
  "term_id": "GO:0030141",
  "gene_symbol": "KLK4",
  "gene": "UniProtKB:Q9Y5K2"
}